{
  "gene_name": "Acetylcholine receptor subunit gamma",
  "gene": "UniProtKB:P07510",
  "gene_symbol": "CHRNG",
  "term_id": "GO:0043005",
  "term_label": "neuron projection"
}